{
  "term_label": "cardiac muscle cell action potential involved in contraction",
  "gene": "UniProtKB:Q14524",
  "term_id": "GO:0086002",
  "gene_name": "Sodium channel protein type 5 subunit alpha",
  "gene_symbol": "SCN5A"
}